complement component C1q receptor activity [GO:0001857] (molecular function) Definition: Combining with the C1q complex, a component of the classical complement cascade, and transmitting the signal from one side of the membrane to the other to initiate a change in cell activity. Relationships: is a type of opsonin receptor activity [GO:0001847]; is a type of complement receptor activity [GO:0004875]; has part complement component C1q complex binding [GO:0001849] Sources: GOC:add, GOC:signaling, ISBN:0781735149